choline sulfotransferase activity [GO:0047754] (molecular function) Relationships: is a type of sulfotransferase activity [GO:0008146] Sources: EC:2.8.2.6, RHEA:21984 Also known as: choline sulphotransferase activity, 3'-phosphoadenylyl-sulfate:choline sulfotransferase activity, choline sulphokinase activity Definition: Catalysis of the reaction: 3'-phospho-5'-adenylyl sulfate + choline = adenosine 3',5'-diphosphate + choline sulfate + H+.